{
  "term_id": "GO:0005886",
  "gene": "UniProtKB:P42679",
  "term_label": "plasma membrane",
  "gene_symbol": "MATK",
  "gene_name": "Megakaryocyte-associated tyrosine-protein kinase"
}